{
  "gene": "UniProtKB:Q04771",
  "term_id": "GO:0007507",
  "gene_symbol": "ACVR1",
  "term_label": "heart development",
  "gene_name": "Activin receptor type-1"
}